{
  "gene_name": "Zinc finger protein 180",
  "gene_symbol": "ZNF180",
  "term_id": "GO:0000981",
  "gene": "UniProtKB:Q9UJW8",
  "term_label": "DNA-binding transcription factor activity, RNA polymerase II-specific"
}